{
  "gene_name": "Transcription factor 15",
  "gene_symbol": "TCF15",
  "term_id": "GO:0000981",
  "term_label": "DNA-binding transcription factor activity, RNA polymerase II-specific",
  "gene": "UniProtKB:Q12870"
}